{
  "gene_name": "Myeloid leukemia factor 1",
  "term_id": "GO:0005737",
  "gene_symbol": "MLF1",
  "gene": "UniProtKB:P58340",
  "term_label": "cytoplasm"
}